{
  "gene_name": "GTP-binding protein Rheb",
  "term_id": "GO:1904263",
  "gene": "UniProtKB:Q15382",
  "term_label": "positive regulation of TORC1 signaling",
  "gene_symbol": "RHEB"
}